{
  "term_id": "GO:0004674",
  "gene_name": "Bromodomain testis-specific protein",
  "gene_symbol": "BRDT",
  "gene": "UniProtKB:Q58F21",
  "term_label": "protein serine/threonine kinase activity"
}